maintenance of protein location in plasma membrane [GO:0072660] (biological process) Relationships: is a type of maintenance of protein location in membrane [GO:0072658]; is part of protein localization to plasma membrane [GO:0072659] Definition: Any process in which a protein is maintained in a specific location in the plasma membrane, and is prevented from moving elsewhere. Sources: GOC:mah